{
  "gene_name": "Alpha-(1,3)-fucosyltransferase 4",
  "gene_symbol": "FUT4",
  "term_label": "Unknown biological process",
  "gene": "UniProtKB:P22083",
  "term_id": "UNKNOWN:0002"
}